{
  "term_id": "GO:0019773",
  "gene_symbol": "PSMA4",
  "gene": "UniProtKB:P25789",
  "term_label": "proteasome core complex, alpha-subunit complex",
  "gene_name": "Proteasome subunit alpha type-4"
}